{
  "term_id": "UNKNOWN:0003",
  "gene_name": "T cell receptor alpha joining 59 (non-functional) (Fragment)",
  "term_label": "Unknown cellular component",
  "gene": "UniProtKB:A0A075B6V9",
  "gene_symbol": "TRAJ59"
}